{
  "term_label": "nucleus",
  "gene": "UniProtKB:O95416",
  "term_id": "GO:0005634",
  "gene_name": "Transcription factor SOX-14",
  "gene_symbol": "SOX14"
}